{
  "gene_symbol": "SPATA31C2",
  "gene": "UniProtKB:B4DYI2",
  "term_id": "UNKNOWN:0002",
  "term_label": "Unknown biological process",
  "gene_name": "Putative spermatogenesis-associated protein 31C2"
}